osteoblast fate commitment [GO:0002051] (biological process) Relationships: is a type of cell fate commitment [GO:0045165]; is part of osteoblast differentiation [GO:0001649] Definition: The commitment of mesenchymal cells to the specific cell fate of an osteoblast. An osteoblast is a bone-forming cell which secretes an extracellular matrix. Hydroxyapatite crystals are then deposited into the matrix to form bone. Sources: GOC:dph